cannabinoid biosynthetic process [GO:1901696] (biological process) Definition: The chemical reactions and pathways resulting in the formation of cannabinoid. Also known as: cannabinoid anabolism, cannabinoid biosynthesis, cannabinoid formation, cannabinoid synthesis Relationships: is a type of biosynthetic process [GO:0009058] Sources: GOC:TermGenie